{
  "gene": "UniProtKB:Q9C0C7",
  "gene_name": "Activating molecule in BECN1-regulated autophagy protein 1",
  "term_label": "ubiquitin-like ligase-substrate adaptor activity",
  "gene_symbol": "AMBRA1",
  "term_id": "GO:1990756"
}